response to histidine [GO:0080052] (biological process) Definition: Any process that results in a change in state or activity of a cell or an organism (in terms of movement, secretion, enzyme production, gene expression, etc.) as a result of a histidine stimulus. References: PMID:15889294 Relationships: is a type of GO:0043200; is_a response to nitrogen compound [GO:1901698]; is a type of response to oxygen-containing compound [GO:1901700] Subtypes: GO:0071232